spindle pole body separation [GO:0110100] (biological process) Note: Note that this term is in the subset of terms that should not be used for direct gene product annotation. Instead, select a child term or, if no appropriate child term exists, please request a new term. Direct annotations to this term may be amended during annotation QC. Subtypes: initial mitotic spindle pole body separation [GO:0000073], initial meiotic spindle pole body separation [GO:0140456] Definition: The release of duplicated spindle pole bodies (SPBs) and their migration away from each other within the nuclear membrane. Duplicated SPBs are connected by a bridge structure that is severed in order to release the SPBs from one another. Following liberation, SPBs diffuse through the nuclear membrane until they are across from each other. SPB separation must take place in order for a bipolar spindle to assemble. Sources: GOC:vw Relationships: is a type of GO:0022402; is part of spindle pole body organization [GO:0051300]